{
  "gene_symbol": "DIRAS3",
  "term_id": "GO:0007264",
  "gene_name": "GTP-binding protein Di-Ras3",
  "gene": "UniProtKB:O95661",
  "term_label": "small GTPase-mediated signal transduction"
}